{
  "term_label": "nucleus",
  "gene": "UniProtKB:Q9HBL8",
  "gene_symbol": "NMRAL1",
  "term_id": "GO:0005634",
  "gene_name": "NmrA-like family domain-containing protein 1"
}